cellulose synthase (UDP-forming) activity [GO:0016760] (molecular function) Sources: EC:2.4.1.12 Also known as: 1,4-beta-D-glucan synthase activity, 1,4-beta-glucan synthase activity, GS-I, UDP-glucose-1,4-beta-glucan glucosyltransferase activity, UDP-glucose-beta-D-glucan glucosyltransferase activity, UDP-glucose-cellulose glucosyltransferase activity, UDP-glucose:1,4-beta-D-glucan 4-beta-D-glucosyltransferase activity, UDPglucose-beta-glucan glucosyltransferase activity, UDPglucose-cellulose glucosyltransferase activity, UDPglucose:1,4-beta-D-glucan 4-beta-D-glucosyltransferase activity, beta-1,4-glucan synthase activity, beta-1,4-glucan synthetase activity, beta-1,4-glucosyltransferase activity, beta-glucan synthase activity, glucan synthase activity, uridine diphosphoglucose-1,4-beta-glucan glucosyltransferase activity, uridine diphosphoglucose-cellulose glucosyltransferase activity Relationships: is a type of cellulose synthase activity [GO:0016759]; is a type of UDP-glucosyltransferase activity [GO:0035251] Definition: Catalysis of the reaction: UDP-glucose + ((1,4)-beta-D-glucosyl)(n) = UDP + ((1,4)-beta-D-glucosyl)(n+1).